{
  "gene_name": "Testis-expressed protein 19",
  "term_label": "nucleus",
  "gene_symbol": "TEX19",
  "term_id": "GO:0005634",
  "gene": "UniProtKB:Q8NA77"
}